{
  "gene_symbol": "TRAJ47",
  "gene": "UniProtKB:A0A075B6Y5",
  "term_label": "Unknown biological process",
  "term_id": "UNKNOWN:0002",
  "gene_name": "T cell receptor alpha joining 47 (Fragment)"
}